{
  "gene_symbol": "ANKRD11",
  "term_id": "GO:0005654",
  "gene": "UniProtKB:Q6UB99",
  "term_label": "nucleoplasm",
  "gene_name": "Ankyrin repeat domain-containing protein 11"
}